{
  "term_label": "UDP-galactose:glucosylceramide beta-1,4-galactosyltransferase activity",
  "term_id": "GO:0008489",
  "gene": "UniProtKB:Q9UBX8",
  "gene_symbol": "B4GALT6",
  "gene_name": "Beta-1,4-galactosyltransferase 6"
}